isopenicillin-N epimerase activity [GO:0045439] (molecular function) Definition: Catalysis of the reaction: isopenicillin N = penicillin N. Sources: EC:5.1.1.17, RHEA:20033 Relationships: is a type of GO:0016855 Also known as: isopenicillin N epimerase activity, penicillin-N 5-amino-5-carboxypentanoyl-epimerase activity